{
  "term_label": "antimicrobial humoral immune response mediated by antimicrobial peptide",
  "term_id": "GO:0061844",
  "gene": "UniProtKB:O95715",
  "gene_name": "C-X-C motif chemokine 14",
  "gene_symbol": "CXCL14"
}